{
  "gene_symbol": "UVRAG",
  "gene": "UniProtKB:Q9P2Y5",
  "gene_name": "UV radiation resistance-associated gene protein",
  "term_id": "GO:0000149",
  "term_label": "SNARE binding"
}